RNA polymerase I core factor complex [GO:0070860] (CC) References: PMID:8702872 Note: Note that, although this complex can be considered analogous to the mammalian transcription factor SL complex, the core factor complex does not include TBP, whereas SL1 does. Definition: A RNA polymerase I-specific transcription factor complex that is required for the transcription of rDNA by RNA polymerase I. In yeast the complex consists of Rrn6p, Rrn7p, and Rrn11p. Relationships: is a type of RNA polymerase I transcription regulator complex [GO:0000120]